{
  "term_label": "signal transduction",
  "gene_symbol": "PHKG2",
  "term_id": "GO:0007165",
  "gene": "UniProtKB:P15735",
  "gene_name": "Phosphorylase b kinase gamma catalytic chain, liver_testis isoform"
}